{
  "term_id": "GO:0071013",
  "gene_name": "Heterogeneous nuclear ribonucleoprotein A1-like 2",
  "gene": "UniProtKB:Q32P51",
  "term_label": "catalytic step 2 spliceosome",
  "gene_symbol": "HNRNPA1L2"
}